{
  "gene_name": "Fibroblast growth factor 23",
  "gene": "UniProtKB:Q9GZV9",
  "term_id": "GO:0043410",
  "gene_symbol": "FGF23",
  "term_label": "positive regulation of MAPK cascade"
}